{
  "gene": "UniProtKB:A0N4Z7",
  "term_label": "Unknown biological process",
  "term_id": "UNKNOWN:0002",
  "gene_symbol": "TRAJ10",
  "gene_name": "Possible J 10 gene (Fragment)"
}